{
  "gene": "UniProtKB:P55084",
  "gene_name": "Trifunctional enzyme subunit beta, mitochondrial",
  "term_label": "acetyl-CoA C-acetyltransferase activity",
  "term_id": "GO:0003985",
  "gene_symbol": "HADHB"
}